axonemal microtubule doublet outer junction [GO:0160114] (cellular component) Relationships: is a type of cellular anatomical structure [GO:0110165]; is part of axonemal doublet microtubule [GO:0097545] Definition: The structure which joins the B1 protofilament of the B tubule to the A10 and A11 protofilaments of the A tubule within an axonemal microtubule doublet. References: PMID:29430673, PMID:37295417 Sources: GOC:krc